{
  "term_id": "UNKNOWN:0002",
  "gene_name": "Putative uncharacterized protein FLJ44553",
  "term_label": "Unknown biological process",
  "gene_symbol": "Q86TA4",
  "gene": "UniProtKB:Q86TA4"
}